{
  "gene": "UniProtKB:Q9NSY0",
  "term_id": "GO:0006974",
  "gene_name": "Nuclear receptor-binding protein 2",
  "term_label": "DNA damage response",
  "gene_symbol": "NRBP2"
}